{
  "gene_symbol": "THAP10",
  "term_label": "Unknown biological process",
  "term_id": "UNKNOWN:0002",
  "gene_name": "THAP domain-containing protein 10",
  "gene": "UniProtKB:Q9P2Z0"
}